type 8 metabotropic glutamate receptor binding [GO:0031805] (molecular function) Sources: GOC:mah, GOC:nln Relationships: is a type of G protein-coupled glutamate receptor binding [GO:0035256] Definition: Binding to a type 8 metabotropic glutamate receptor. Also known as: type 8 metabotropic glutamate receptor ligand